interleukin-27 receptor binding [GO:0045523] (molecular function) Definition: Binding to an interleukin-27 receptor. Sources: GOC:go_curators Also known as: IL-27, interleukin-27 receptor ligand Relationships: is a type of cytokine receptor binding [GO:0005126]